alpha-glucosidase activity [GO:0090599] (molecular function) Relationships: is a type of glucosidase activity [GO:0015926] Subtypes: GO:0004135, glucan 1,4-alpha-glucosidase activity [GO:0004339], alpha-1,4-glucosidase activity [GO:0004558], Glc3Man9GlcNAc2 oligosaccharide glucosidase activity [GO:0004573], oligo-1,6-glucosidase activity [GO:0004574], GO:0004575, glucan 1,3-alpha-glucosidase activity [GO:0033919], GO:0033933, GO:0043896, glucan endo-1,3-alpha-glucosidase activity [GO:0051118], Glc2Man9GlcNAc2 oligosaccharide glucosidase activity [GO:0106407] Sources: GOC:tb Definition: Catalysis of the hydrolysis of terminal, non-reducing alpha-linked alpha-D-glucose residue with release of alpha-D-glucose.